{
  "gene_symbol": "CDHR5",
  "gene": "UniProtKB:Q9HBB8",
  "gene_name": "Cadherin-related family member 5",
  "term_label": "plasma membrane",
  "term_id": "GO:0005886"
}